2-methylcitrate synthase activity [GO:0050440] (MF) Sources: RHEA:23780 Relationships: is a type of acyltransferase activity, acyl groups converted into alkyl on transfer [GO:0046912] Definition: Catalysis of the reaction: H2O + oxaloacetate + propanoyl-CoA = (2R,3S)-2-methylcitrate + CoA + H+. Also known as: 2-methylcitrate oxaloacetate-lyase activity, MCS activity, methylcitrate synthase activity, methylcitrate synthetase activity, propanoyl-CoA:oxaloacetate C-propanoyltransferase (thioester-hydrolysing, 1-carboxyethyl-forming)